{
  "gene_name": "Vesicle transport protein GOT1A",
  "gene_symbol": "GOLT1A",
  "term_label": "membrane",
  "gene": "UniProtKB:Q6ZVE7",
  "term_id": "GO:0016020"
}